{
  "gene": "UniProtKB:Q96Q91",
  "term_label": "regulation of intracellular pH",
  "gene_name": "Anion exchange protein 4",
  "gene_symbol": "SLC4A9",
  "term_id": "GO:0051453"
}